regulation of inner ear auditory receptor cell fate specification [GO:0042669] (biological process) Sources: GOC:go_curators Definition: Any process that mediates the specification of a cell into an auditory hair cell. Relationships: is a type of regulation of cell fate specification [GO:0042659]; is a type of GO:0045607; regulates auditory receptor cell fate specification [GO:0042667] Subtypes: negative regulation of auditory receptor cell fate specification [GO:0009999] Also known as: regulation of auditory hair cell fate specification